{
  "gene_name": "Ran-binding protein 9",
  "term_id": "GO:0030674",
  "gene": "UniProtKB:Q96S59",
  "gene_symbol": "RANBP9",
  "term_label": "protein-macromolecule adaptor activity"
}